{
  "gene_name": "Costars family protein ABRACL",
  "gene": "UniProtKB:Q9P1F3",
  "gene_symbol": "ABRACL",
  "term_id": "UNKNOWN:0003",
  "term_label": "Unknown cellular component"
}